{
  "gene_symbol": "RPS19",
  "gene_name": "Small ribosomal subunit protein eS19",
  "term_id": "GO:0003735",
  "term_label": "structural constituent of ribosome",
  "gene": "UniProtKB:P39019"
}